{
  "gene": "UniProtKB:A0A6Q8PFD8",
  "gene_name": "Uncharacterized protein",
  "term_label": "Unknown cellular component",
  "term_id": "UNKNOWN:0003",
  "gene_symbol": "A0A6Q8PFD8"
}